protein catabolic process [GO:0030163] (biological process) Relationships: is a type of macromolecule catabolic process [GO:0009057]; is a type of protein metabolic process [GO:0019538] Sources: GOC:mah Definition: The chemical reactions and pathways resulting in the breakdown of a protein by the destruction of the native, active configuration, with or without the hydrolysis of peptide bonds. Note: This term refers to the breakdown of mature proteins. For cleavage events involved in generating a mature protein from a precursor, consider instead the term 'protein maturation ; GO:0051604' and its children. Regulation: regulated by regulation of protein catabolic process [GO:0042176]; RO_0002212 by GO:0042177; positively regulated by positive regulation of protein catabolic process [GO:0045732] Subtypes: glycoprotein catabolic process [GO:0006516], protein catabolic process in the vacuole [GO:0007039], epidermal growth factor catabolic process [GO:0007174], PSII associated light-harvesting complex II catabolic process [GO:0010304], proteasomal protein catabolic process [GO:0010498], protein denaturation [GO:0030164], GO:0032802, mitochondrial protein catabolic process [GO:0035694], histone catabolic process [GO:0036205], lipoprotein catabolic process [GO:0042159], hemoglobin catabolic process [GO:0042540], rhodopsin catabolic process [GO:0046155], GO:0061684, protein catabolic process at synapse [GO:0140246], insulin catabolic process [GO:1901143] Also known as: cellular protein breakdown, cellular protein catabolic process, cellular protein catabolism, cellular protein degradation, protein breakdown, protein catabolism, protein degradation, multicellular organismal protein catabolic process, pheromone catabolic process, pheromone catabolism